{
  "gene_name": "Olfactory receptor 51E2",
  "term_label": "plasma membrane",
  "gene_symbol": "OR51E2",
  "gene": "UniProtKB:Q9H255",
  "term_id": "GO:0005886"
}